{
  "term_label": "plasma membrane",
  "term_id": "GO:0005886",
  "gene_symbol": "NMUR1",
  "gene": "UniProtKB:Q9HB89",
  "gene_name": "Neuromedin-U receptor 1"
}